{
  "gene": "UniProtKB:Q9Y6M5",
  "gene_name": "Proton-coupled zinc antiporter SLC30A1",
  "gene_symbol": "SLC30A1",
  "term_label": "endoplasmic reticulum",
  "term_id": "GO:0005783"
}